bacteriocin metabolic process [GO:0046224] (biological process) Also known as: bacteriocin metabolism Relationships: is a type of toxin metabolic process [GO:0009404]; is a type of GO:0043603 Sources: GOC:ai Definition: The chemical reactions and pathways involving bacteriocins, any of a heterogeneous group of polypeptide antibiotics that are secreted by certain bacterial strains and are able to kill cells of other susceptible (frequently related) strains after adsorption at specific receptors on the cell surface. They include the colicins, and their mechanisms of action vary. Subtypes: bacteriocin biosynthetic process [GO:0030152], bacteriocin catabolic process [GO:0046225]